receptor catabolic process [GO:0032801] (biological process) Definition: The chemical reactions and pathways resulting in the breakdown of a receptor molecule, a macromolecule that undergoes combination with a hormone, neurotransmitter, drug or intracellular messenger to initiate a change in cell function. Sources: GOC:mah Also known as: receptor breakdown, receptor catabolism, receptor degradation Relationships: is a type of macromolecule catabolic process [GO:0009057]; is_a receptor metabolic process [GO:0043112] Subtypes: low-density lipoprotein particle receptor catabolic process [GO:0032802], Wnt receptor catabolic process [GO:0038018], G protein-coupled receptor catabolic process [GO:1990172] Regulation: regulated by regulation of receptor catabolic process [GO:2000644]; negatively regulated by GO:2000645; positively regulated by positive regulation of receptor catabolic process [GO:2000646]